{
  "term_id": "UNKNOWN:0001",
  "gene": "UniProtKB:Q16617",
  "term_label": "Unknown molecular function",
  "gene_name": "Protein NKG7",
  "gene_symbol": "NKG7"
}